{
  "gene_symbol": "NAGLU",
  "term_label": "alpha-N-acetylglucosaminidase activity",
  "term_id": "GO:0004561",
  "gene_name": "Alpha-N-acetylglucosaminidase",
  "gene": "UniProtKB:P54802"
}